{
  "gene": "UniProtKB:Q9H6D8",
  "gene_symbol": "FNDC4",
  "term_id": "UNKNOWN:0002",
  "gene_name": "Fibronectin type III domain-containing protein 4",
  "term_label": "Unknown biological process"
}